{
  "term_label": "DNA-binding transcription factor activity, RNA polymerase II-specific",
  "gene": "UniProtKB:Q15562",
  "gene_symbol": "TEAD2",
  "term_id": "GO:0000981",
  "gene_name": "Transcriptional enhancer factor TEF-4"
}